{
  "gene_name": "Nuclear receptor subfamily 4 group A member 2",
  "term_label": "dopaminergic neuron differentiation",
  "term_id": "GO:0071542",
  "gene": "UniProtKB:P43354",
  "gene_symbol": "NR4A2"
}